{
  "gene_symbol": "DUX4L3",
  "term_id": "GO:0005634",
  "term_label": "nucleus",
  "gene_name": "Double homeobox protein 4-like protein 3",
  "gene": "UniProtKB:P0CJ86"
}